{
  "gene_name": "Copine-1",
  "gene": "UniProtKB:Q99829",
  "gene_symbol": "CPNE1",
  "term_id": "GO:0071277",
  "term_label": "cellular response to calcium ion"
}